{
  "term_label": "Unknown molecular function",
  "gene_name": "Reticulon-2",
  "gene": "UniProtKB:O75298",
  "gene_symbol": "RTN2",
  "term_id": "UNKNOWN:0001"
}